{
  "gene": "UniProtKB:Q9H227",
  "gene_symbol": "GBA3",
  "term_id": "GO:0046477",
  "gene_name": "Cytosolic beta-glucosidase",
  "term_label": "glycosylceramide catabolic process"
}